{
  "term_id": "UNKNOWN:0001",
  "gene": "UniProtKB:Q8N131",
  "gene_symbol": "TMEM123",
  "term_label": "Unknown molecular function",
  "gene_name": "Porimin"
}